{
  "gene": "UniProtKB:P30414",
  "gene_name": "NK-tumor recognition protein",
  "term_label": "nucleus",
  "term_id": "GO:0005634",
  "gene_symbol": "NKTR"
}